neuroblast delamination [GO:0060234] (biological process) Relationships: is a type of delamination [GO:0060232] Sources: GOC:dph Definition: The negative regulation of cell adhesion process in which a neuroblast splits off of a neurectodermal sheet.